germ-line stem cell population maintenance [GO:0030718] (BP) Subtypes: male germ-line stem cell population maintenance [GO:0036098], female germ-line stem cell population maintenance [GO:0036099] Sources: ISBN:0879694238 Definition: Any process by which an organism or tissue maintains a population of germ-line stem cells. Relationships: is a type of stem cell population maintenance [GO:0019827]